{
  "term_id": "GO:0031902",
  "term_label": "late endosome membrane",
  "gene_symbol": "ATP13A3",
  "gene": "UniProtKB:Q9H7F0",
  "gene_name": "Polyamine-transporting ATPase 13A3"
}